{
  "gene_name": "Cytosolic arginine sensor for mTORC1 subunit 2",
  "term_id": "GO:1903577",
  "gene_symbol": "CASTOR2",
  "gene": "UniProtKB:A6NHX0",
  "term_label": "cellular response to L-arginine"
}